tyrosine N-monooxygenase activity [GO:0050370] (molecular function) Sources: MetaCyc:TYROSINE-N-MONOOXYGENASE-RXN Relationships: is a type of oxidoreductase activity, acting on paired donors, with incorporation or reduction of molecular oxygen, NAD(P)H as one donor, and incorporation of one atom of oxygen [GO:0016709] Also known as: L-tyrosine,NADPH:oxygen oxidoreductase (N-hydroxylating), tyrosine N-hydroxylase activity, CYP79A1 activity Definition: Catalysis of the reaction: tyrosine + O2 + NADPH + H+ = N-hydroxytyrosine + NADP+ + H2O.